{
  "gene_symbol": "RHOXF2B",
  "term_id": "GO:0005634",
  "gene_name": "Rhox homeobox family member 2B",
  "gene": "UniProtKB:P0C7M4",
  "term_label": "nucleus"
}